{
  "term_id": "GO:0008191",
  "gene_name": "Retinoic acid receptor responder protein 1",
  "term_label": "metalloendopeptidase inhibitor activity",
  "gene": "UniProtKB:P49788",
  "gene_symbol": "RARRES1"
}